negative regulation of maternal process involved in parturition [GO:1904302] (biological process) Relationships: is a type of negative regulation of multicellular organismal process [GO:0051241]; is a type of regulation of maternal process involved in parturition [GO:1904301]; is a type of negative regulation of reproductive process [GO:2000242]; RO_0002212 GO:0060137 Also known as: down regulation of maternal process involved in parturition, down-regulation of maternal process involved in parturition, downregulation of maternal process involved in parturition, inhibition of maternal process involved in parturition References: PMID:1849751 Sources: GOC:TermGenie, GO_REF:0000058 Definition: Any process that stops, prevents or reduces the frequency, rate or extent of maternal process involved in parturition.